{
  "gene": "UniProtKB:Q008S8",
  "term_label": "Unknown biological process",
  "term_id": "UNKNOWN:0002",
  "gene_symbol": "ECT2L",
  "gene_name": "Epithelial cell-transforming sequence 2 oncogene-like"
}